intestinal cholesterol absorption [GO:0030299] (biological process) Definition: Uptake of cholesterol into the blood by absorption from the small intestine. Relationships: is a type of GO:0098856; is part of lipid digestion [GO:0044241] Regulation: regulated by regulation of intestinal cholesterol absorption [GO:0030300]; negatively regulated by negative regulation of intestinal cholesterol absorption [GO:0045796]; positively regulated by GO:0045797 Sources: GOC:mah